10-hydroxydihydrosanguinarine 10-O-methyltransferase activity [GO:0030779] (molecular function) Sources: EC:2.1.1.119, RHEA:18541 Also known as: S-adenosyl-L-methionine:10-hydroxydihydrosanguinarine 10-O-methyltransferase activity Definition: Catalysis of the reaction: 10-hydroxydihydrosanguinarine + S-adenosyl-L-methionine(1+) = S-adenosyl-L-homocysteine + dihydrochelirubine + H+. Relationships: is_a GO:0008757